{
  "gene": "UniProtKB:Q15836",
  "gene_name": "Vesicle-associated membrane protein 3",
  "term_label": "SNAP receptor activity",
  "term_id": "GO:0005484",
  "gene_symbol": "VAMP3"
}